late endosomal microautophagy [GO:0061738] (biological process) Definition: The autophagy process by which cytosolic proteins targeted for degradation are tagged with a chaperone and are directly transferred into and degraded in a late endosomal compartment. References: PMID:21238931 Sources: GOC:PARL, GOC:autophagy, GOC:dph, GOC:pad Relationships: is a type of GO:0016237